{
  "term_label": "positive regulation of DNA-templated transcription",
  "gene": "UniProtKB:Q8TF47",
  "gene_name": "Zinc finger protein 90 homolog",
  "gene_symbol": "ZFP90",
  "term_id": "GO:0045893"
}